ABC-type betaine transporter activity [GO:0031458] (MF) Sources: GOC:mlg Relationships: is a type of GO:0140359 Definition: Catalysis of the reaction: ATP + H2O + a betaine(out) = ADP + phosphate + a betaine(in). Also known as: ABC-type betaine transmembrane transporter activity, ATP-dependent betaine transporter activity, betaine-transporting ATPase activity, betaine ABC transporter, ATPase-coupled betaine transporter activity